{
  "gene_name": "Cadherin-related family member 1",
  "term_label": "cell adhesion molecule binding",
  "gene_symbol": "CDHR1",
  "gene": "UniProtKB:Q96JP9",
  "term_id": "GO:0050839"
}